phagocytic vesicle lumen [GO:0097013] (cellular component) Relationships: is a type of GO:0071682; is part of phagocytic vesicle [GO:0045335] Definition: The volume enclosed by the membrane of a phagocytic vesicle. Subtypes: GO:0062113, phagolysosome vesicle lumen [GO:0106174] Sources: GOC:rs